{
  "gene_name": "N-terminal kinase-like protein",
  "gene": "UniProtKB:Q96KG9",
  "gene_symbol": "SCYL1",
  "term_id": "UNKNOWN:0002",
  "term_label": "Unknown biological process"
}